{
  "gene_name": "Cytokine SCM-1 beta",
  "term_id": "GO:0005615",
  "gene": "UniProtKB:Q9UBD3",
  "term_label": "extracellular space",
  "gene_symbol": "XCL2"
}